{
  "gene": "UniProtKB:Q5EBL8",
  "term_label": "pore complex assembly",
  "gene_symbol": "PDZD11",
  "term_id": "GO:0046931",
  "gene_name": "PDZ domain-containing protein 11"
}